(+)-camphor catabolic process [GO:0019383] (biological process) Definition: The chemical reactions and pathways resulting in the breakdown of (+)-camphor, a bicyclic monoterpene ketone. Also known as: (+)-camphor breakdown, (+)-camphor catabolism, (+)-camphor degradation Relationships: is a type of monoterpenoid catabolic process [GO:0016100]; is a type of ketone catabolic process [GO:0042182] Sources: MetaCyc:P601-PWY